clearance of cells from fusion plate by epithelial to mesenchymal transition [GO:0060886] (biological process) Definition: The process of epithelial to mesenchymal transition that contributes to the shaping of the semicircular canal by effectively removing epithelial cells from the fusion plate, forming the loops of the canals. Relationships: is a type of GO:0001837; is a type of clearance of cells from fusion plate [GO:0060884] Sources: GOC:dph, GOC:sdb_2009, GOC:tb